{
  "gene_symbol": "TTC23",
  "term_id": "UNKNOWN:0002",
  "term_label": "Unknown biological process",
  "gene": "UniProtKB:Q5W5X9",
  "gene_name": "Tetratricopeptide repeat protein 23"
}